{
  "gene_name": "Uncharacterized protein C2orf78",
  "gene": "UniProtKB:A6NCI8",
  "term_id": "UNKNOWN:0002",
  "gene_symbol": "C2orf78",
  "term_label": "Unknown biological process"
}